{
  "gene_symbol": "CASP2",
  "gene": "UniProtKB:P42575",
  "gene_name": "Caspase-2",
  "term_label": "intrinsic apoptotic signaling pathway in response to DNA damage",
  "term_id": "GO:0008630"
}